{
  "gene": "UniProtKB:Q9BVL4",
  "term_id": "UNKNOWN:0003",
  "term_label": "Unknown cellular component",
  "gene_name": "Protein adenylyltransferase SelO, mitochondrial",
  "gene_symbol": "SELENOO"
}